{
  "gene_symbol": "GHR",
  "gene": "UniProtKB:P10912",
  "gene_name": "Growth hormone receptor",
  "term_id": "GO:0060396",
  "term_label": "growth hormone receptor signaling pathway"
}